inositol-1,3,4,6-tetrakisphosphate 6-phosphatase activity [GO:0052830] (molecular function) Relationships: is a type of GO:0052743 Sources: GOC:ai Definition: Catalysis of the reaction: inositol-1,3,4,6-tetrakisphosphate + H2O = inositol-1,3,4-trisphosphate + phosphate.